protein localization to ciliary membrane [GO:1903441] (BP) Subtypes: GO:0097500 References: PMID:22139371 Sources: GOC:TermGenie, GOC:cilia, GOC:krc, GO_REF:0000087 Regulation: regulated by GO:1903567; negatively regulated by negative regulation of protein localization to ciliary membrane [GO:1903568]; RO_0002213 by positive regulation of protein localization to ciliary membrane [GO:1903569] Relationships: is_a protein localization to cilium [GO:0061512]; is a type of protein localization to membrane [GO:0072657]; is a type of protein localization to cell periphery [GO:1990778] Definition: A process in which a protein is transported to, or maintained in, a location within a ciliary membrane. Also known as: protein localisation in ciliary membrane, protein localisation to ciliary membrane, protein localization in ciliary membrane